{
  "term_id": "GO:0045773",
  "gene_name": "Immunoglobulin superfamily containing leucine-rich repeat protein 2",
  "gene_symbol": "ISLR2",
  "term_label": "positive regulation of axon extension",
  "gene": "UniProtKB:Q6UXK2"
}